{
  "term_id": "UNKNOWN:0002",
  "term_label": "Unknown biological process",
  "gene": "UniProtKB:Q8TAB5",
  "gene_symbol": "C1orf216",
  "gene_name": "UPF0500 protein C1orf216"
}